{
  "gene_name": "Myosin-7B",
  "term_label": "Unknown biological process",
  "gene": "UniProtKB:A7E2Y1",
  "term_id": "UNKNOWN:0002",
  "gene_symbol": "MYH7B"
}